{
  "term_id": "UNKNOWN:0003",
  "gene_symbol": "GCDH",
  "gene_name": "Glutaryl-CoA dehydrogenase, mitochondrial",
  "term_label": "Unknown cellular component",
  "gene": "UniProtKB:Q92947"
}